{
  "term_id": "GO:0051607",
  "gene_name": "BCL2_adenovirus E1B 19 kDa protein-interacting protein 3-like",
  "gene": "UniProtKB:O60238",
  "term_label": "defense response to virus",
  "gene_symbol": "BNIP3L"
}